{
  "gene": "UniProtKB:P55017",
  "gene_name": "Solute carrier family 12 member 3",
  "term_label": "potassium ion homeostasis",
  "gene_symbol": "SLC12A3",
  "term_id": "GO:0055075"
}